{
  "term_label": "Unknown molecular function",
  "gene": "UniProtKB:Q7L804",
  "gene_name": "Rab11 family-interacting protein 2",
  "term_id": "UNKNOWN:0001",
  "gene_symbol": "RAB11FIP2"
}